{
  "term_id": "GO:0005763",
  "gene_name": "Small ribosomal subunit protein uS5m",
  "gene": "UniProtKB:P82675",
  "term_label": "mitochondrial small ribosomal subunit",
  "gene_symbol": "MRPS5"
}